{
  "term_id": "GO:0000978",
  "term_label": "RNA polymerase II cis-regulatory region sequence-specific DNA binding",
  "gene": "UniProtKB:Q12772",
  "gene_symbol": "SREBF2",
  "gene_name": "Sterol regulatory element-binding protein 2"
}